{
  "term_label": "Unknown molecular function",
  "gene_name": "Tumor necrosis factor receptor superfamily member 17",
  "term_id": "UNKNOWN:0001",
  "gene_symbol": "TNFRSF17",
  "gene": "UniProtKB:Q02223"
}